{
  "gene_name": "Growth hormone-inducible transmembrane protein",
  "term_id": "GO:0007007",
  "term_label": "inner mitochondrial membrane organization",
  "gene_symbol": "GHITM",
  "gene": "UniProtKB:Q9H3K2"
}